{
  "term_label": "protein serine/threonine kinase activity",
  "gene_name": "Serine_threonine-protein kinase 38",
  "gene": "UniProtKB:Q15208",
  "gene_symbol": "STK38",
  "term_id": "GO:0004674"
}